{
  "gene": "UniProtKB:Q9BZW5",
  "term_id": "GO:0005765",
  "gene_name": "Transmembrane 6 superfamily member 1",
  "gene_symbol": "TM6SF1",
  "term_label": "lysosomal membrane"
}